{
  "gene": "UniProtKB:Q8IZ63",
  "gene_name": "Proline-rich protein 22",
  "term_id": "UNKNOWN:0003",
  "term_label": "Unknown cellular component",
  "gene_symbol": "PRR22"
}